{
  "term_id": "UNKNOWN:0001",
  "gene_symbol": "ZNF414",
  "gene": "UniProtKB:Q96IQ9",
  "gene_name": "Zinc finger protein 414",
  "term_label": "Unknown molecular function"
}